cetraxate benzylesterase activity [GO:0047741] (molecular function) Relationships: is a type of carboxylic ester hydrolase activity [GO:0052689] Sources: EC:3.1.1.70, RHEA:23460 Definition: Catalysis of the reaction: benzyl cetraxate + H2O = benzyl alcohol + cetraxate + H+. Also known as: cetraxate-benzyl-ester benzylhydrolase activity